solanapyrone synthase activity [GO:0033190] (molecular function) Relationships: is_a cyclase activity [GO:0009975] Definition: Catalysis of the cyclization of double bonds in prosolanapyrone II to form (-)-solanapyrone A. References: PMID:9659400 Sources: GOC:cb